{
  "gene_name": "Keratin-associated protein 16-1",
  "term_id": "UNKNOWN:0002",
  "term_label": "Unknown biological process",
  "gene": "UniProtKB:A8MUX0",
  "gene_symbol": "KRTAP16-1"
}